{
  "term_label": "cis-regulatory region sequence-specific DNA binding",
  "gene_name": "RNA polymerase II elongation factor ELL",
  "term_id": "GO:0000987",
  "gene_symbol": "ELL",
  "gene": "UniProtKB:P55199"
}